{
  "gene_name": "Neuronal acetylcholine receptor subunit alpha-10",
  "term_label": "detection of mechanical stimulus involved in sensory perception of sound",
  "gene_symbol": "CHRNA10",
  "gene": "UniProtKB:Q9GZZ6",
  "term_id": "GO:0050910"
}